{
  "gene_symbol": "ELMO3",
  "gene_name": "Engulfment and cell motility protein 3",
  "term_id": "GO:0005085",
  "gene": "UniProtKB:Q96BJ8",
  "term_label": "guanyl-nucleotide exchange factor activity"
}